{
  "term_label": "synaptic cleft",
  "term_id": "GO:0043083",
  "gene_symbol": "C1QL4",
  "gene": "UniProtKB:Q86Z23",
  "gene_name": "Complement C1q-like protein 4"
}